{
  "gene_name": "Retinol dehydrogenase 5",
  "term_label": "Unknown cellular component",
  "gene_symbol": "RDH5",
  "term_id": "UNKNOWN:0003",
  "gene": "UniProtKB:Q92781"
}